{
  "gene_name": "UBX domain-containing protein 2A",
  "gene_symbol": "UBXN2A",
  "term_label": "nucleus",
  "gene": "UniProtKB:P68543",
  "term_id": "GO:0005634"
}